{
  "gene_name": "Protein phosphatase 1 regulatory subunit 3B",
  "gene_symbol": "PPP1R3B",
  "gene": "UniProtKB:Q86XI6",
  "term_label": "regulation of glycogen biosynthetic process",
  "term_id": "GO:0005979"
}